{
  "term_id": "GO:0016324",
  "gene_name": "Partitioning defective 6 homolog alpha",
  "term_label": "apical plasma membrane",
  "gene_symbol": "PARD6A",
  "gene": "UniProtKB:Q9NPB6"
}